{
  "gene_name": "Zinc finger protein 560",
  "term_id": "GO:0000981",
  "term_label": "DNA-binding transcription factor activity, RNA polymerase II-specific",
  "gene_symbol": "ZNF560",
  "gene": "UniProtKB:Q96MR9"
}